{
  "gene": "UniProtKB:Q9H114",
  "gene_name": "Cystatin-like 1",
  "term_label": "Unknown cellular component",
  "gene_symbol": "CSTL1",
  "term_id": "UNKNOWN:0003"
}